{
  "gene_name": "Nuclear factor of activated T-cells, cytoplasmic 2",
  "gene": "UniProtKB:Q13469",
  "term_label": "transcription regulator complex",
  "gene_symbol": "NFATC2",
  "term_id": "GO:0005667"
}